{
  "gene_name": "Ras-related protein Rab-3C",
  "gene": "UniProtKB:Q96E17",
  "term_label": "synaptic vesicle",
  "gene_symbol": "RAB3C",
  "term_id": "GO:0008021"
}